{
  "gene_symbol": "CEP43",
  "gene": "UniProtKB:O95684",
  "term_id": "GO:0005813",
  "gene_name": "Centrosomal protein 43",
  "term_label": "centrosome"
}